{
  "term_id": "GO:0061630",
  "gene": "UniProtKB:Q86Y01",
  "gene_symbol": "DTX1",
  "term_label": "ubiquitin protein ligase activity",
  "gene_name": "E3 ubiquitin-protein ligase DTX1"
}